5-dehydro-2-deoxyphosphogluconate aldolase activity [GO:0047441] (MF) Also known as: 5-dehydro-2-deoxy-D-gluconate-6-phosphate malonate-semialdehyde-lyase (pyruvate-forming), 5-dehydro-2-deoxy-D-gluconate-6-phosphate malonate-semialdehyde-lyase activity, phospho-5-dehydro-2-deoxygluconate aldolase activity, phospho-5-keto-2-deoxygluconate aldolase activity Relationships: is a type of aldehyde-lyase activity [GO:0016832] Definition: Catalysis of the reaction: 6-phospho-5-dehydro-2-deoxy-D-gluconate = 3-oxopropanoate + glycerone phosphate. Sources: EC:4.1.2.29, RHEA:13177